{
  "term_label": "Unknown cellular component",
  "gene_symbol": "CD55",
  "gene_name": "Complement decay-accelerating factor",
  "gene": "UniProtKB:P08174",
  "term_id": "UNKNOWN:0003"
}